interleukin-3 binding [GO:0019978] (molecular function) Definition: Binding to interleukin-3. Relationships: is a type of GO:0019838; is a type of GO:0019955 Also known as: IL-3 binding Sources: GOC:jl